metal ion transmembrane transporter activity [GO:0046873] (molecular function) Relationships: is a type of GO:0008324; is part of GO:0030001 Also known as: heavy metal ion porter activity, heavy metal ion transporter activity, heavy metal ion:hydrogen symporter activity, heavy metal-exporting ATPase activity, high affinity metal ion uptake transporter activity, low affinity metal ion uptake transporter activity Definition: Enables the transfer of metal ions from one side of a membrane to the other. Sources: GOC:ai Subtypes: potassium ion transmembrane transporter activity [GO:0015079], sodium ion transmembrane transporter activity [GO:0015081], GO:0015085, GO:0015094, magnesium ion transmembrane transporter activity [GO:0015095], GO:0046915, metal cation:monoatomic cation antiporter activity [GO:0140828]